{
  "gene_symbol": "PLAC8",
  "term_id": "GO:0045944",
  "gene": "UniProtKB:Q9NZF1",
  "gene_name": "Placenta-specific gene 8 protein",
  "term_label": "positive regulation of transcription by RNA polymerase II"
}